anthranilate catabolic process [GO:0043421] (BP) Definition: The chemical reactions and pathways resulting in the breakdown of anthranilate (2-aminobenzoate). Sources: GOC:jl Also known as: 2-aminobenzoate breakdown, 2-aminobenzoate catabolic process, 2-aminobenzoate degradation, anthranilate breakdown, anthranilate catabolism, anthranilate degradation, 2-aminobenzoate catabolism, anthranilic acid catabolic process, anthranilic acid catabolism, ortho-aminobenzoic acid catabolic process, ortho-aminobenzoic acid catabolism Relationships: is a type of aromatic amino acid family catabolic process [GO:0009074]; is a type of xenobiotic catabolic process [GO:0042178]; is a type of anthranilate metabolic process [GO:0043420]; is a type of monocarboxylic acid catabolic process [GO:0072329]